{
  "gene_symbol": "IGLL1",
  "term_id": "GO:0003823",
  "gene_name": "Immunoglobulin lambda-like polypeptide 1",
  "gene": "UniProtKB:P15814",
  "term_label": "antigen binding"
}